{
  "term_id": "GO:0000028",
  "gene_symbol": "RPSA",
  "gene": "UniProtKB:P08865",
  "gene_name": "Small ribosomal subunit protein uS2",
  "term_label": "ribosomal small subunit assembly"
}